membrane protein dislocase activity [GO:0140567] (molecular function) References: PMID:24821790, PMID:28712723, PMID:32973005 Definition: The activity of removing a protein from a membrane, by binding to a transmembrane helical fragment of a tail-anchored protein and releasing it from the the hydrophobic region of one or both lipid bilayers. The reaction is driven by ATP hydrolysis. Also known as: transmembrane helix dislocase
transmembrane protein dislocase activity Relationships: is a type of protein transporter activity [GO:0140318]; is a type of ATP-dependent activity [GO:0140657]